extrinsic component of presynaptic endosome membrane [GO:0099007] (cellular component) Sources: GOC:autophagy, GOC:mf Relationships: is a type of GO:0031313; is part of presynaptic endosome membrane [GO:0098954] Definition: The component of the presynaptic endosome membrane consisting of gene products and protein complexes that are loosely bound to one of its surfaces, but not integrated into the hydrophobic region.